{
  "gene_name": "Spermatogenesis-associated protein 48",
  "term_label": "spermatogenesis",
  "term_id": "GO:0007283",
  "gene": "UniProtKB:A4D263",
  "gene_symbol": "SPMIP7"
}